{
  "gene_name": "Ceramide synthase 4",
  "term_label": "endoplasmic reticulum",
  "gene": "UniProtKB:Q9HA82",
  "gene_symbol": "CERS4",
  "term_id": "GO:0005783"
}